{
  "gene_name": "Nuclear receptor-interacting protein 3",
  "gene_symbol": "NRIP3",
  "term_id": "GO:0004190",
  "gene": "UniProtKB:Q9NQ35",
  "term_label": "aspartic-type endopeptidase activity"
}